{
  "gene_name": "Uncharacterized protein C11orf97",
  "gene": "UniProtKB:A0A1B0GVM6",
  "gene_symbol": "C11orf97",
  "term_id": "UNKNOWN:0001",
  "term_label": "Unknown molecular function"
}